{
  "gene_symbol": "LMNA",
  "gene_name": "Prelamin-A_C",
  "term_label": "nuclear envelope organization",
  "term_id": "GO:0006998",
  "gene": "UniProtKB:P02545"
}